{
  "gene_symbol": "TRIM16L",
  "term_label": "Unknown biological process",
  "gene_name": "Tripartite motif-containing protein 16-like protein",
  "gene": "UniProtKB:Q309B1",
  "term_id": "UNKNOWN:0002"
}